acetylcholine receptor regulator activity [GO:0030548] (molecular function) Relationships: is a type of GO:0099602; regulates acetylcholine receptor activity [GO:0015464] Subtypes: acetylcholine receptor activator activity [GO:0030549], GO:0030550 Sources: GOC:mah Definition: Interacting (directly or indirectly) with acetylcholine receptors such that the proportion of receptors in the active form is changed.